{
  "gene_name": "Protein KRI1 homolog",
  "term_id": "GO:0030686",
  "gene": "UniProtKB:Q8N9T8",
  "gene_symbol": "KRI1",
  "term_label": "90S preribosome"
}